{
  "gene_symbol": "S100A7",
  "term_label": "calcium ion binding",
  "gene_name": "Protein S100-A7",
  "term_id": "GO:0005509",
  "gene": "UniProtKB:P31151"
}